{
  "term_label": "kynurenine metabolic process",
  "gene_symbol": "KMO",
  "gene_name": "Kynurenine 3-monooxygenase",
  "gene": "UniProtKB:O15229",
  "term_id": "GO:0070189"
}